{
  "gene": "UniProtKB:Q14696",
  "gene_symbol": "MESD",
  "term_label": "low-density lipoprotein particle receptor binding",
  "gene_name": "LRP chaperone MESD",
  "term_id": "GO:0050750"
}